delta-carotene catabolic process [GO:1901823] (BP) References: PMID:8837512 Sources: GOC:TermGenie, GOC:yaf, MetaCyc:PWY-5946, UniPathway:UPA00801 Also known as: delta-carotene breakdown, delta-carotene catabolism, delta-carotene degradation Relationships: is a type of carotenoid catabolic process [GO:0016118]; is a type of GO:0016121 Definition: The chemical reactions and pathways resulting in the breakdown of delta-carotene.